negative regulation of tetrapyrrole catabolic process [GO:1901405] (biological process) Subtypes: negative regulation of chlorophyll catabolic process [GO:1903647] Sources: GOC:TermGenie, GOC:mengo_curators Also known as: down regulation of tetrapyrrole breakdown, down regulation of tetrapyrrole catabolic process, down regulation of tetrapyrrole catabolism, down regulation of tetrapyrrole degradation, down-regulation of tetrapyrrole breakdown, down-regulation of tetrapyrrole catabolic process, down-regulation of tetrapyrrole catabolism, down-regulation of tetrapyrrole degradation, downregulation of tetrapyrrole breakdown, downregulation of tetrapyrrole catabolic process, downregulation of tetrapyrrole catabolism, downregulation of tetrapyrrole degradation, inhibition of tetrapyrrole breakdown, inhibition of tetrapyrrole catabolism, inhibition of tetrapyrrole degradation, negative regulation of tetrapyrrole breakdown, negative regulation of tetrapyrrole catabolism, negative regulation of tetrapyrrole degradation, inhibition of tetrapyrrole catabolic process Relationships: is_a negative regulation of catabolic process [GO:0009895]; is a type of regulation of tetrapyrrole catabolic process [GO:1901404]; negatively regulates tetrapyrrole catabolic process [GO:0033015] Definition: Any process that stops, prevents or reduces the frequency, rate or extent of tetrapyrrole catabolic process.